{
  "term_label": "Unknown biological process",
  "gene_symbol": "C2orf42",
  "term_id": "UNKNOWN:0002",
  "gene": "UniProtKB:Q9NWW7",
  "gene_name": "Uncharacterized protein C2orf42"
}